{
  "gene_name": "Anaphase-promoting complex subunit 16",
  "gene_symbol": "ANAPC16",
  "term_label": "protein ubiquitination",
  "gene": "UniProtKB:Q96DE5",
  "term_id": "GO:0016567"
}